{
  "gene_symbol": "PLA2G10",
  "term_label": "phosphatidylglycerol metabolic process",
  "gene_name": "Group 10 secretory phospholipase A2",
  "gene": "UniProtKB:O15496",
  "term_id": "GO:0046471"
}